polyuridylation-dependent decapping of nuclear-transcribed mRNA [GO:0036450] (biological process) Also known as: uridylation-dependent decapping of nuclear-transcribed mRNA Relationships: is a type of deadenylation-independent decapping of nuclear-transcribed mRNA [GO:0031087]; is part of polyuridylation-dependent mRNA catabolic process [GO:1990074] References: PMID:19430462 Sources: GOC:vw Definition: Cleavage of the 5'-cap of a nuclear-transcribed mRNA that has been modified by the enzymatic addition of a sequence of uridylyl residues (polyuridylation) at the 3' end.